galactose import across plasma membrane [GO:0140425] (biological process) Definition: The directed movement of galactose from outside of a cell, across the plasma membrane and into the cytosol. Relationships: is a type of galactose transmembrane transport [GO:0015757]; is a type of hexose import across plasma membrane [GO:0140271] References: PMID:21621292, PMID:23254763